{
  "gene_symbol": "ZBTB24",
  "term_id": "GO:0003700",
  "gene_name": "Zinc finger and BTB domain-containing protein 24",
  "gene": "UniProtKB:O43167",
  "term_label": "DNA-binding transcription factor activity"
}